{
  "gene": "UniProtKB:Q15699",
  "gene_name": "ALX homeobox protein 1",
  "term_id": "GO:0048666",
  "term_label": "neuron development",
  "gene_symbol": "ALX1"
}